{
  "term_id": "UNKNOWN:0002",
  "gene_symbol": "MANSC1",
  "gene": "UniProtKB:Q9H8J5",
  "gene_name": "MANSC domain-containing protein 1",
  "term_label": "Unknown biological process"
}